ATPase-coupled transmembrane transporter activity [GO:0042626] (molecular function) Definition: Primary active transporter of a solute across a membrane, via the reaction: ATP + H2O = ADP + phosphate, to directly drive the transport of a substance across a membrane. The transport protein may be transiently phosphorylated (P-type transporters), or not (ABC-type transporters and other families of transporters). Primary active transport occurs up the solute's concentration gradient and is driven by a primary energy source. Subtypes: ATPase-coupled phosphate ion transmembrane transporter activity [GO:0015415], GO:0015446, GO:0015450, ATPase-coupled monoatomic cation transmembrane transporter activity [GO:0019829], ATPase-coupled urea transmembrane transporter activity [GO:0033221], GO:0033225, GO:0033284, ATPase-coupled lipid transmembrane transporter activity [GO:0034040], ATPase-coupled ion transmembrane transporter activity [GO:0042625], ATPase-coupled antimonite transmembrane transporter activity [GO:0042961], P-type transmembrane transporter activity [GO:0140358], ABC-type transporter activity [GO:0140359], ATPase-coupled lipo-chitin oligosaccharide transmembrane transporter activity [GO:1901514] Relationships: is a type of primary active transmembrane transporter activity [GO:0015399]; is a type of ATP-dependent activity [GO:0140657] Sources: GOC:mtg_transport, ISBN:0815340729 Also known as: ATPase activity, coupled to movement of substances, P-P-bond-hydrolysis-driven transmembrane transporter activity, P-P-bond-hydrolysis-driven transporter, ATP-coupled transmembrane transporter activity, ATP-dependent transmembrane transporter activity, ATPase activity, coupled to transmembrane movement of substances, hydrolase activity, acting on acid anhydrides, catalyzing transmembrane movement of substances